IgM immunoglobulin complex [GO:0071753] (cellular component) Definition: A protein complex composed of two identical immunoglobulin heavy chains of the IgM isotype and two identical immunoglobulin light chains, held together by disulfide bonds, and in its circulating form complexed with J chain in polymeric forms. An IgM immunoglobulin complex may be embedded in the plasma membrane or present in the extracellular space, in mucosal areas or other tissues, or circulating in the blood or lymph. References: PMID:20176268 Sources: GOC:add, ISBN:0781765196 Note: Note that an IgM immunoglobulin complex has the function of antigen binding if a suitable antigen is available. Relationships: is a type of immunoglobulin complex [GO:0019814] Subtypes: GO:0071754, IgM B cell receptor complex [GO:0071755]